regulation of double-strand break repair via homologous recombination [GO:0010569] (biological process) Subtypes: regulation of double-strand break repair via break-induced replication [GO:1901591], GO:1905168, negative regulation of double-strand break repair via homologous recombination [GO:2000042] Definition: Any process that modulates the frequency, rate or extent of the error-free repair of a double-strand break in DNA in which the broken DNA molecule is repaired using homologous sequences. Relationships: is a type of regulation of DNA recombination [GO:0000018]; is a type of GO:2000779; regulates double-strand break repair via homologous recombination [GO:0000724] Sources: GOC:dph, GOC:jp, GOC:tb